{
  "term_id": "GO:0061630",
  "gene_name": "Probable E3 ubiquitin-protein ligase makorin-3",
  "gene_symbol": "MKRN3",
  "gene": "UniProtKB:Q13064",
  "term_label": "ubiquitin protein ligase activity"
}